{
  "term_id": "GO:0045202",
  "gene_name": "Zinc finger MYND domain-containing protein 19",
  "gene": "UniProtKB:Q96E35",
  "gene_symbol": "ZMYND19",
  "term_label": "synapse"
}